{
  "term_label": "triglyceride catabolic process",
  "gene_name": "Lipoprotein lipase",
  "term_id": "GO:0019433",
  "gene": "UniProtKB:P06858",
  "gene_symbol": "LPL"
}